{
  "term_label": "Unknown cellular component",
  "term_id": "UNKNOWN:0003",
  "gene_name": "Transmembrane inner ear expressed protein",
  "gene": "UniProtKB:Q8NEW7",
  "gene_symbol": "TMIE"
}